viral genome packaging [GO:0019072] (biological process) Definition: The encapsulation of the viral genome within the capsid. Sources: ISBN:0121585336 Subtypes: viral DNA genome packaging [GO:0019073], viral RNA genome packaging [GO:0019074] Relationships: is_a viral process [GO:0016032]; is part of GO:0019068